{
  "term_id": "GO:0032281",
  "gene_name": "Monoacylglycerol lipase ABHD6",
  "term_label": "AMPA glutamate receptor complex",
  "gene_symbol": "ABHD6",
  "gene": "UniProtKB:Q9BV23"
}